{
  "term_id": "UNKNOWN:0003",
  "gene": "UniProtKB:Q7L5A3",
  "gene_symbol": "ATOSB",
  "gene_name": "Atos homolog protein B",
  "term_label": "Unknown cellular component"
}